{
  "gene_name": "AKT-interacting protein",
  "gene": "UniProtKB:Q9H8T0",
  "term_label": "ubiquitin conjugating enzyme activity",
  "gene_symbol": "AKTIP",
  "term_id": "GO:0061631"
}